positive regulation of lens epithelial cell proliferation [GO:2001111] (biological process) Sources: GOC:obol Relationships: is a type of GO:0050679; is a type of regulation of lens epithelial cell proliferation [GO:2001109]; positively regulates lens epithelial cell proliferation [GO:0097166] Definition: Any process that activates or increases the frequency, rate or extent of lens epithelial cell proliferation.